{
  "gene_name": "Dual specificity protein phosphatase 16",
  "gene": "UniProtKB:Q9BY84",
  "term_id": "UNKNOWN:0002",
  "gene_symbol": "DUSP16",
  "term_label": "Unknown biological process"
}